{
  "gene_symbol": "PAX8",
  "gene": "UniProtKB:Q06710",
  "term_id": "GO:0000981",
  "gene_name": "Paired box protein Pax-8",
  "term_label": "DNA-binding transcription factor activity, RNA polymerase II-specific"
}